7-deoxyloganetic acid glucosyltransferase activity [GO:0102970] (molecular function) Relationships: is_a hexosyltransferase activity [GO:0016758] Definition: Catalysis of the reaction: UDP-alpha-D-glucose + 7-deoxyloganetate = H+ + 7-deoxyloganate + UDP. Sources: EC:2.4.1.323, GOC:pz